{
  "term_label": "S-adenosylmethionine biosynthetic process",
  "gene_name": "S-adenosylmethionine synthase isoform type-2",
  "term_id": "GO:0006556",
  "gene": "UniProtKB:P31153",
  "gene_symbol": "MAT2A"
}